{
  "gene_symbol": "VPS37A",
  "term_label": "protein targeting to membrane",
  "gene": "UniProtKB:Q8NEZ2",
  "gene_name": "Vacuolar protein sorting-associated protein 37A",
  "term_id": "GO:0006612"
}